response to amitrole [GO:0072722] (biological process) Definition: Any process that results in a change in state or activity of a cell or an organism (in terms of movement, secretion, enzyme production, gene expression, etc.) as a result of an amitrole stimulus. Also known as: response to 3-amino-1,2,4-triazole Sources: GOC:mah Relationships: is a type of response to nitrogen compound [GO:1901698] Subtypes: cellular response to amitrole [GO:0072723]